O-acetylhomoserine sulfhydrylase activity [GO:0051009] (molecular function) Sources: MetaCyc:ACETYLHOMOSER-CYS-RXN, RHEA:27822 Also known as: homocysteine synthase Relationships: is a type of O-acetylhomoserine aminocarboxypropyltransferase activity [GO:0003961]; is a type of carbon-oxygen lyase activity [GO:0016835] Definition: Catalysis of the reaction: O-acetyl-L-homoserine + hydrogen sulfide = homocysteine + acetate.